{
  "gene_name": "Monocarboxylate transporter 9",
  "gene_symbol": "SLC16A9",
  "gene": "UniProtKB:Q7RTY1",
  "term_id": "GO:0005886",
  "term_label": "plasma membrane"
}